{
  "term_label": "positive regulation of neuron apoptotic process",
  "gene_name": "Caspase-6",
  "term_id": "GO:0043525",
  "gene_symbol": "CASP6",
  "gene": "UniProtKB:P55212"
}